{
  "gene": "UniProtKB:O00217",
  "gene_symbol": "NDUFS8",
  "term_id": "GO:0045271",
  "term_label": "respiratory chain complex I",
  "gene_name": "NADH dehydrogenase [ubiquinone] iron-sulfur protein 8, mitochondrial"
}